{
  "gene_symbol": "CDC42SE1",
  "gene_name": "CDC42 small effector protein 1",
  "term_label": "plasma membrane",
  "gene": "UniProtKB:Q9NRR8",
  "term_id": "GO:0005886"
}